1-acylglycerol-3-phosphate O-acyltransferase activity [GO:0003841] (molecular function) Sources: EC:2.3.1.51, GOC:ab Relationships: is a type of GO:0016411; is a type of GO:0042171 Also known as: 1-acyl-sn-glycerol-3-phosphate acyltransferase activity, lysophosphatidate acyltransferase activity, 1-acyl-sn-glycero-3-phosphate acyltransferase activity, 1-acyl-sn-glycerol 3-phosphate acyltransferase activity, 1-acylglycero-3-phosphate acyltransferase activity, 1-acylglycerolphosphate acyltransferase activity, 1-acylglycerophosphate acyltransferase activity, acyl-CoA:1-acyl-sn-glycerol-3-phosphate 2-O-acyltransferase activity, lysophosphatidic acid-acyltransferase activity Definition: Catalysis of the reaction: acyl-CoA + 1-acyl-sn-glycerol-3-phosphate = CoA + 1,2-diacyl-sn-glycerol-3-phosphate.